{
  "gene_name": "ER membrane protein complex subunit 3",
  "gene": "UniProtKB:Q9P0I2",
  "term_id": "GO:0032977",
  "gene_symbol": "EMC3",
  "term_label": "membrane insertase activity"
}